{
  "term_label": "Unknown biological process",
  "term_id": "UNKNOWN:0002",
  "gene_symbol": "EXOC1L",
  "gene_name": "Exocyst complex component 1-like",
  "gene": "UniProtKB:A0A1B0GW35"
}